{
  "term_label": "regulation of transcription by RNA polymerase II",
  "term_id": "GO:0006357",
  "gene": "UniProtKB:A6NM28",
  "gene_name": "Zinc finger protein 92 homolog",
  "gene_symbol": "ZFP92"
}